{
  "gene": "UniProtKB:A0A0C4DH59",
  "term_label": "cell surface receptor signaling pathway",
  "gene_symbol": "TRBV5-4",
  "term_id": "GO:0007166",
  "gene_name": "T cell receptor beta variable 5-4"
}